{
  "term_label": "calcium-dependent phospholipid binding",
  "gene": "UniProtKB:Q9BQS2",
  "gene_symbol": "SYT15",
  "gene_name": "Synaptotagmin-15",
  "term_id": "GO:0005544"
}